{
  "gene_name": "Trans-Golgi network integral membrane protein 2",
  "gene_symbol": "TGOLN2",
  "term_id": "GO:0030140",
  "gene": "UniProtKB:O43493",
  "term_label": "trans-Golgi network transport vesicle"
}